{
  "gene_name": "Mothers against decapentaplegic homolog 4",
  "term_id": "GO:0000981",
  "term_label": "DNA-binding transcription factor activity, RNA polymerase II-specific",
  "gene": "UniProtKB:Q13485",
  "gene_symbol": "SMAD4"
}